{
  "term_id": "GO:0030154",
  "gene_symbol": "CAV1",
  "term_label": "cell differentiation",
  "gene_name": "Caveolin-1",
  "gene": "UniProtKB:Q03135"
}